{
  "gene": "UniProtKB:O76090",
  "gene_symbol": "BEST1",
  "term_label": "chloride transmembrane transport",
  "term_id": "GO:1902476",
  "gene_name": "Bestrophin-1"
}